{
  "term_label": "cytoplasmic exosome (RNase complex)",
  "gene": "UniProtKB:Q5RKV6",
  "gene_symbol": "EXOSC6",
  "gene_name": "Exosome complex component MTR3",
  "term_id": "GO:0000177"
}